{
  "term_id": "UNKNOWN:0001",
  "gene_symbol": "TRAV5",
  "term_label": "Unknown molecular function",
  "gene": "UniProtKB:A0A0B4J249",
  "gene_name": "T cell receptor alpha variable 5"
}